{
  "term_id": "GO:1905515",
  "gene_symbol": "TMEM216",
  "gene": "UniProtKB:Q9P0N5",
  "gene_name": "Transmembrane protein 216",
  "term_label": "non-motile cilium assembly"
}